negative regulation of L-proline import across plasma membrane [GO:1905736] (biological process) Definition: Any process that stops, prevents or reduces the frequency, rate or extent of L-proline import across plasma membrane. References: PMID:24344203 Sources: GOC:TermGenie, GO_REF:0000058 Relationships: is a type of negative regulation of proline import across plasma membrane [GO:1902835]; is a type of regulation of L-proline import across plasma membrane [GO:1905735]; negatively regulates GO:1904271